protein storage [GO:0140089] (biological process) Relationships: is a type of GO:0170062 Definition: The accumulation and maintenance in cells of proteins. Protein reserves can be accumulated during early developmental stages for mobilization and utilization at later stages of development. References: PMID:37922900